regulation of blood microparticle formation [GO:2000332] (biological process) Subtypes: negative regulation of blood microparticle formation [GO:2000333], positive regulation of blood microparticle formation [GO:2000334], GO:2000335 Sources: GOC:BHF, GOC:mah Definition: Any process that modulates the frequency, rate or extent of blood microparticle formation. Relationships: is a type of regulation of developmental process [GO:0050793]; is a type of regulation of cellular component organization [GO:0051128]; RO_0002211 blood microparticle formation [GO:0072564] Also known as: regulation of microparticle generation, regulation of microparticle release